{
  "gene": "UniProtKB:O60260",
  "term_label": "ubiquitin ligase complex",
  "gene_symbol": "PRKN",
  "term_id": "GO:0000151",
  "gene_name": "E3 ubiquitin-protein ligase parkin"
}